{
  "gene_symbol": "SSR1",
  "term_label": "Unknown biological process",
  "term_id": "UNKNOWN:0002",
  "gene_name": "Translocon-associated protein subunit alpha",
  "gene": "UniProtKB:P43307"
}